{
  "term_label": "RNA polymerase II cis-regulatory region sequence-specific DNA binding",
  "gene_name": "Zinc finger protein 611",
  "gene_symbol": "ZNF611",
  "term_id": "GO:0000978",
  "gene": "UniProtKB:Q8N823"
}